(S)-6-hydroxynicotine oxidase activity [GO:0018531] (molecular function) Also known as: 6-hydroxy-L-nicotine oxidase activity, L-6-hydroxynicotine oxidase activity, (S)-6-hydroxynicotine:oxygen oxidoreductase activity, 6-hydroxy-L-nicotine:oxygen oxidoreductase activity Definition: Catalysis of the reaction: (S)-6-hydroxynicotine + H2O + O2 = 6-hydroxypseudooxynicotine + H2O2. Relationships: is a type of GO:0019116 Sources: EC:1.5.3.5, RHEA:11880